positive regulation of meiotic sister chromatid arm separation [GO:0062041] (biological process) References: PMID:20383139 Definition: Any process that increases the rate or extent of meiotic sister chromatid arm separation, the cell cycle process in which sister chromatid arms are physically detached from each other during meiosis. Relationships: is a type of positive regulation of meiotic chromosome separation [GO:1905134]; positively regulates meiotic sister chromatid arm separation [GO:0051755]